{
  "term_label": "Unknown cellular component",
  "gene_name": "Arylsulfatase L",
  "gene": "UniProtKB:P51690",
  "term_id": "UNKNOWN:0003",
  "gene_symbol": "ARSL"
}